{
  "term_id": "GO:0007399",
  "term_label": "nervous system development",
  "gene": "UniProtKB:Q06710",
  "gene_symbol": "PAX8",
  "gene_name": "Paired box protein Pax-8"
}